{
  "gene": "UniProtKB:Q9UGM3",
  "term_id": "GO:0050830",
  "gene_name": "Deleted in malignant brain tumors 1 protein",
  "term_label": "defense response to Gram-positive bacterium",
  "gene_symbol": "DMBT1"
}